{
  "gene_name": "Long-chain fatty acid transport protein 2",
  "term_label": "bile acid metabolic process",
  "gene_symbol": "SLC27A2",
  "term_id": "GO:0008206",
  "gene": "UniProtKB:O14975"
}